{
  "term_label": "nucleolus",
  "gene": "UniProtKB:Q9UGY1",
  "gene_name": "Nucleolar protein 12",
  "term_id": "GO:0005730",
  "gene_symbol": "NOL12"
}